interleukin-34 production [GO:0150155] (biological process) References: PMID:26754294 Sources: GOC:aruk Definition: The appearance of interleukin-34 due to biosynthesis or secretion following a cellular stimulus, resulting in an increase in its intracellular or extracellular levels. Relationships: is a type of cytokine production [GO:0001816] Regulation: regulated by regulation of interleukin-34 production [GO:0150157]; positively regulated by positive regulation of interleukin-34 production [GO:0150158]; negatively regulated by negative regulation of interleukin-34 production [GO:0150159]